{
  "term_label": "epithelial cell differentiation",
  "gene": "UniProtKB:O76014",
  "gene_name": "Keratin, type I cuticular Ha7",
  "term_id": "GO:0030855",
  "gene_symbol": "KRT37"
}